{
  "gene": "UniProtKB:Q9Y2I6",
  "term_id": "GO:0034454",
  "gene_name": "Ninein-like protein",
  "gene_symbol": "NINL",
  "term_label": "microtubule anchoring at centrosome"
}